melanosome [GO:0042470] (cellular component) References: PMID:11584301 Sources: GOC:jl Definition: A tissue-specific, membrane-bounded cytoplasmic organelle within which melanin pigments are synthesized and stored. Melanosomes are synthesized in melanocyte cells. Relationships: is a type of pigment granule [GO:0048770]